{
  "gene_name": "COP9 signalosome complex subunit 2",
  "gene_symbol": "COPS2",
  "term_id": "GO:0008180",
  "gene": "UniProtKB:P61201",
  "term_label": "COP9 signalosome"
}